{
  "term_id": "GO:0007030",
  "gene_name": "Golgin subfamily A member 8A",
  "gene_symbol": "GOLGA8A",
  "gene": "UniProtKB:A7E2F4",
  "term_label": "Golgi organization"
}